{
  "term_id": "GO:0005737",
  "gene_symbol": "ISCA1",
  "term_label": "cytoplasm",
  "gene": "UniProtKB:Q9BUE6",
  "gene_name": "Iron-sulfur cluster assembly 1 homolog, mitochondrial"
}